{
  "term_label": "Unknown biological process",
  "gene_symbol": "SACS",
  "gene": "UniProtKB:Q9NZJ4",
  "term_id": "UNKNOWN:0002",
  "gene_name": "Sacsin"
}